negative regulation of mechanoreceptor differentiation [GO:0045632] (biological process) Also known as: down regulation of mechanoreceptor differentiation, down-regulation of mechanoreceptor differentiation, downregulation of mechanoreceptor differentiation, inhibition of mechanoreceptor differentiation Definition: Any process that stops, prevents, or reduces the frequency, rate or extent of mechanoreceptor differentiation. Relationships: is a type of regulation of mechanoreceptor differentiation [GO:0045631]; is a type of negative regulation of neuron differentiation [GO:0045665]; negatively regulates GO:0042490 Sources: GOC:go_curators Subtypes: negative regulation of inner ear receptor cell differentiation [GO:2000981]